antiporter activity [GO:0015297] (molecular function) Subtypes: acetylcholine:proton antiporter activity [GO:0005278], GO:0005452, succinate:fumarate antiporter activity [GO:0005469], ATP:ADP antiporter activity [GO:0005471], carnitine:O-acyl-L-carnitine antiporter activity [GO:0005476], folate:monoatomic anion antiporter activity [GO:0008518], GTP:GDP antiporter activity [GO:0010292], cycloheximide:proton antiporter activity [GO:0015309], GO:0015310, monoamine:proton antiporter activity [GO:0015311], GO:0015312, GO:0015325, cystine:glutamate antiporter activity [GO:0015327], oxoglutarate:malate antiporter activity [GO:0015367], putrescine:ornithine antiporter activity [GO:0015496], citrate:succinate antiporter activity [GO:0015515], tartrate:succinate antiporter activity [GO:0015516], tetracycline:proton antiporter activity [GO:0015520], acridine:proton antiporter activity [GO:0042962], GO:0043858, agmatine:putrescine antiporter activity [GO:0043861], arginine:agmatine antiporter activity [GO:0043862], lysine:cadaverine antiporter activity [GO:0043872], (R)-carnitine:4-(trimethylammonio)butanoate antiporter activity [GO:0044667], GO:0045119, GO:0062057, aspartate:alanine antiporter activity [GO:0070906], L-histidine:histamine antiporter activity [GO:0070907], tyrosine:tyramine antiporter activity [GO:0070908], glutamate:gamma-aminobutyric acid antiporter activity [GO:0070909], GO:0099520, monoatomic ion antiporter activity involved in regulation of postsynaptic membrane potential [GO:0099580], L-lysine:L-arginine antiporter activity [GO:0106439], GO:0140812, urate:monoatomic anion antiporter activity [GO:0140813], metal cation:monoatomic cation antiporter activity [GO:0140828], bicarbonate:monoatomic anion antiporter activity [GO:0140829], amino acid:monoatomic cation antiporter activity [GO:0140848], GO:0140968, S-adenosyl-L-methionine:S-adenosyl-L-homocysteine antiporter activity [GO:0180003], broad specificity neutral L-amino acid:basic L-amino acid antiporter activity [GO:0180009], citrate:2-oxoglutarate antiporter activity [GO:0180056] Also known as: exchanger, porter, countertransporter activity, exchange transporter activity, solute:solute antiporter activity, ion antiporter activity, antiport, solute:solute exchange Relationships: is a type of secondary active transmembrane transporter activity [GO:0015291] Definition: Enables the active transport of a solute across a membrane by a mechanism whereby two or more species are transported in opposite directions in a tightly coupled process not directly linked to a form of energy other than chemiosmotic energy. The reaction is: solute A(out) + solute B(in) = solute A(in) + solute B(out). References: PMID:10839820 Sources: GOC:mtg_transport, ISBN:0815340729